{
  "term_id": "GO:0005737",
  "term_label": "cytoplasm",
  "gene_name": "Serine_threonine-protein kinase OSR1",
  "gene": "UniProtKB:O95747",
  "gene_symbol": "OXSR1"
}